{
  "gene": "UniProtKB:Q06203",
  "term_label": "purine nucleotide biosynthetic process",
  "gene_name": "Amidophosphoribosyltransferase",
  "gene_symbol": "PPAT",
  "term_id": "GO:0006164"
}